{
  "gene_name": "Putative uncharacterized protein encoded by LINC00208",
  "gene": "UniProtKB:Q96KT6",
  "gene_symbol": "LINC00208",
  "term_label": "Unknown cellular component",
  "term_id": "UNKNOWN:0003"
}